{
  "gene": "UniProtKB:Q6ZQQ2",
  "gene_name": "Spermatogenesis-associated protein 31D1",
  "term_id": "UNKNOWN:0001",
  "gene_symbol": "SPATA31D1",
  "term_label": "Unknown molecular function"
}